B cell affinity maturation [GO:0002344] (biological process) Also known as: B lymphocyte affinity maturation, B-cell affinity maturation, B-lymphocyte affinity maturation Sources: GOC:jal, GO_REF:0000022, ISBN:0781735149 Definition: The process in which B cells produce antibodies with increased antigen affinity. This is accomplished by somatic hypermutation and selection for B cells which produce higher affinity antibodies to antigen. Relationships: is a type of peripheral B cell selection [GO:0002343]; is part of immunoglobulin production involved in immunoglobulin-mediated immune response [GO:0002381]